octopamine biosynthetic process [GO:0006589] (biological process) Relationships: is a type of biogenic amine biosynthetic process [GO:0042401]; is a type of alcohol biosynthetic process [GO:0046165]; is a type of phenol-containing compound biosynthetic process [GO:0046189]; is a type of octopamine metabolic process [GO:0046333] Sources: ISBN:0198506732 Also known as: octopamine anabolism, octopamine biosynthesis, octopamine formation, octopamine synthesis Definition: The chemical reactions and pathways resulting in the formation of octopamine, 1-(p-hydroxyphenyl)-2-aminoethanol. The D enantiomer is about one-tenth as active as norepinephrine and is found in the salivary glands of Octopus and Eledone species.